tissue remodeling [GO:0048771] (biological process) Definition: The reorganization or renovation of existing tissues. This process can either change the characteristics of a tissue such as in blood vessel remodeling, or result in the dynamic equilibrium of a tissue such as in bone remodeling. Sources: GOC:ebc Also known as: tissue remodelling Relationships: is a type of multicellular organismal process [GO:0032501] Subtypes: blood vessel remodeling [GO:0001974], clearance of damaged tissue involved in inflammatory response wound healing [GO:0002247], atrial ventricular junction remodeling [GO:0003294], erythrocyte clearance [GO:0034102], bone remodeling [GO:0046849], mammary gland involution [GO:0060056], GO:0061843, GO:0097709 Regulation: regulated by regulation of tissue remodeling [GO:0034103]; negatively regulated by GO:0034104; positively regulated by positive regulation of tissue remodeling [GO:0034105]